{
  "gene_name": "Septin-4",
  "term_id": "GO:0017157",
  "gene_symbol": "SEPTIN4",
  "term_label": "regulation of exocytosis",
  "gene": "UniProtKB:O43236"
}